{
  "gene": "UniProtKB:Q93091",
  "term_label": "innate immune response",
  "term_id": "GO:0045087",
  "gene_name": "Ribonuclease K6",
  "gene_symbol": "RNASE6"
}